{
  "term_label": "fructose:sodium symporter activity",
  "gene_symbol": "SLC5A10",
  "term_id": "GO:0140930",
  "gene_name": "Sodium_mannose cotransporter SLC5A10",
  "gene": "UniProtKB:A0PJK1"
}